{
  "gene": "UniProtKB:A0A0C4DH29",
  "gene_symbol": "IGHV1-3",
  "term_id": "UNKNOWN:0003",
  "term_label": "Unknown cellular component",
  "gene_name": "Immunoglobulin heavy variable 1-3"
}